negative regulation of transcription of nucleolar large rRNA by RNA polymerase I [GO:1901837] (biological process) Relationships: is a type of GO:0016479; is a type of regulation of transcription of nucleolar large rRNA by RNA polymerase I [GO:1901836]; negatively regulates nucleolar large rRNA transcription by RNA polymerase I [GO:0042790] Also known as: down regulation of transcription of nuclear large rRNA transcript from RNA polymerase I promoter, down regulation of transcription of nuclear rRNA large Pol I transcript, down-regulation of transcription of nuclear large rRNA transcript from RNA polymerase I promoter, down-regulation of transcription of nuclear rRNA large Pol I transcript, downregulation of transcription of nuclear large rRNA transcript from RNA polymerase I promoter, downregulation of transcription of nuclear rRNA large Pol I transcript, inhibition of transcription of nuclear rRNA large Pol I transcript, negative regulation of transcription of nuclear large rRNA transcript from RNA polymerase I promoter, negative regulation of transcription of nuclear rRNA large Pol I transcript, inhibition of transcription of nuclear large rRNA transcript from RNA polymerase I promoter Sources: GOC:TermGenie, GOC:sart Definition: Any process that stops, prevents or reduces the frequency, rate or extent of transcription of nuclear large rRNA transcript mediated by RNA polymerase I.